positive regulation of post-translational protein modification [GO:1901875] (biological process) Also known as: activation of PTM, activation of post-translational amino acid modification, activation of post-translational modification, activation of posttranslational amino acid modification, activation of posttranslational modification, activation of posttranslational protein modification, positive regulation of PTM, positive regulation of post-translational amino acid modification, positive regulation of post-translational modification, positive regulation of posttranslational amino acid modification, positive regulation of posttranslational modification, positive regulation of posttranslational protein modification, up regulation of PTM, up regulation of post-translational amino acid modification, up regulation of post-translational modification, up regulation of post-translational protein modification, up regulation of posttranslational amino acid modification, up regulation of posttranslational modification, up regulation of posttranslational protein modification, up-regulation of PTM, up-regulation of post-translational amino acid modification, up-regulation of post-translational modification, up-regulation of post-translational protein modification, up-regulation of posttranslational amino acid modification, up-regulation of posttranslational modification, up-regulation of posttranslational protein modification, upregulation of PTM, upregulation of post-translational amino acid modification, upregulation of post-translational modification, upregulation of post-translational protein modification, upregulation of posttranslational amino acid modification, upregulation of posttranslational modification, upregulation of posttranslational protein modification, activation of post-translational protein modification Definition: Any process that activates or increases the frequency, rate or extent of post-translational protein modification. Relationships: is a type of GO:0031401; is a type of GO:1901873; positively regulates GO:0043687 References: PMID:21209915 Sources: GOC:TermGenie, GOC:yaf Subtypes: positive regulation of protein modification by small protein conjugation or removal [GO:1903322]